dimethylaniline-N-oxide aldolase activity [GO:0047864] (molecular function) Relationships: is a type of aldehyde-lyase activity [GO:0016832] Definition: Catalysis of the reaction: N,N-dimethylaniline N-oxide = N-methylaniline + formaldehyde. Sources: EC:4.1.2.24, RHEA:19321 Also known as: N,N-dimethylaniline-N-oxide formaldehyde-lyase (N-methylaniline-forming), N,N-dimethylaniline-N-oxide formaldehyde-lyase activity, microsomal N-oxide dealkylase activity, microsomal oxidase II